{
  "gene_name": "Phosphatase and actin regulator 3",
  "gene_symbol": "PHACTR3",
  "term_label": "actin binding",
  "term_id": "GO:0003779",
  "gene": "UniProtKB:Q96KR7"
}